{
  "term_label": "regulation of G protein-coupled receptor signaling pathway",
  "gene": "UniProtKB:Q9Y2K6",
  "term_id": "GO:0008277",
  "gene_name": "Ubiquitin carboxyl-terminal hydrolase 20",
  "gene_symbol": "USP20"
}